{
  "term_id": "GO:0005886",
  "term_label": "plasma membrane",
  "gene_name": "Toll_interleukin-1 receptor domain-containing adapter protein",
  "gene_symbol": "TIRAP",
  "gene": "UniProtKB:P58753"
}